menaquinone metabolic process [GO:0009233] (biological process) Subtypes: GO:0009234, GO:0042361 Relationships: is a type of ketone metabolic process [GO:0042180] Definition: The chemical reactions and pathways involving any of the menaquinones, quinone-derived compounds synthesized by intestinal bacteria. Structurally, menaquinones consist of a methylated naphthoquinone ring structure and side chains composed of a variable number of unsaturated isoprenoid residues. Menaquinones have vitamin K activity and are known as vitamin K2. Also known as: menaquinone metabolism, menatetrenone metabolic process, menatetrenone metabolism, multiprenylmenaquinone metabolic process, multiprenylmenaquinone metabolism, vitamin K2 metabolic process, vitamin K2 metabolism References: PMID:6127606, PMID:8642453 Sources: GOC:jl